{
  "term_id": "UNKNOWN:0001",
  "gene": "UniProtKB:Q6ZTR6",
  "gene_name": "Putative uncharacterized protein ZNF516-DT",
  "gene_symbol": "ZNF516-DT",
  "term_label": "Unknown molecular function"
}